regulation of protein folding in endoplasmic reticulum [GO:0060904] (biological process) Definition: Any process that modulates the rate, frequency or extent of the protein folding process that takes place in the endoplasmic reticulum (ER). Secreted, plasma membrane and organelle proteins are folded in the ER, assisted by chaperones and foldases (protein disulphide isomerases), and additional factors required for optimal folding (ATP, Ca2+ and an oxidizing environment to allow disulfide bond formation). Sources: GOC:dph, GOC:tb Relationships: is a type of regulation of protein folding [GO:1903332]; regulates protein folding in endoplasmic reticulum [GO:0034975]